{
  "term_id": "GO:0000981",
  "gene_symbol": "MEF2A",
  "gene": "UniProtKB:Q02078",
  "gene_name": "Myocyte-specific enhancer factor 2A",
  "term_label": "DNA-binding transcription factor activity, RNA polymerase II-specific"
}